ubiquinone binding [GO:0048039] (molecular function) Definition: Binding to ubiquinone, a quinone derivative with a tail of isoprene units. Relationships: is a type of GO:0048038 Also known as: coenzyme Q binding, coenzyme Q6 binding Sources: GOC:jid, ISBN:0582227089 Subtypes: GO:1900995